{
  "gene": "UniProtKB:Q96S53",
  "gene_name": "Dual specificity testis-specific protein kinase 2",
  "gene_symbol": "TESK2",
  "term_id": "GO:0030036",
  "term_label": "actin cytoskeleton organization"
}